seed abscission [GO:0097548] (biological process) Relationships: is a type of abscission [GO:0009838] Definition: The controlled shedding of a seed. Sources: GOC:lmo